regulation of striated muscle tissue development [GO:0016202] (biological process) Relationships: is_a GO:0048634; is a type of regulation of muscle tissue development [GO:1901861]; regulates striated muscle tissue development [GO:0014706] Sources: GOC:go_curators Definition: Any process that modulates the frequency, rate or extent of striated muscle development. Subtypes: negative regulation of striated muscle tissue development [GO:0045843], GO:0045844, regulation of skeletal muscle tissue development [GO:0048641], regulation of cardiac muscle tissue development [GO:0055024]